{
  "gene_name": "Epididymal sperm-binding protein 1",
  "gene": "UniProtKB:Q96BH3",
  "term_id": "GO:0009986",
  "gene_symbol": "ELSPBP1",
  "term_label": "cell surface"
}